{
  "gene_name": "Neural cell adhesion molecule 1",
  "gene": "UniProtKB:P13591",
  "gene_symbol": "NCAM1",
  "term_id": "UNKNOWN:0001",
  "term_label": "Unknown molecular function"
}